regulation of tRNA export from nucleus [GO:2000238] (biological process) Sources: GOC:mah Also known as: regulation of tRNA export from cell nucleus, regulation of tRNA export out of nucleus, regulation of tRNA transport from nucleus to cytoplasm, regulation of tRNA-nucleus export Relationships: is_a GO:0046831; is a type of regulation of ribonucleoprotein complex localization [GO:2000197]; RO_0002211 tRNA export from nucleus [GO:0006409] Subtypes: GO:2000239, positive regulation of tRNA export from nucleus [GO:2000240] Definition: Any process that modulates the frequency, rate or extent of tRNA export from nucleus.